{
  "gene_name": "Osteopetrosis-associated transmembrane protein 1",
  "gene": "UniProtKB:Q86WC4",
  "gene_symbol": "OSTM1",
  "term_label": "cytosol",
  "term_id": "GO:0005829"
}